regulation of immunoglobulin mediated immune response [GO:0002889] (BP) Definition: Any process that modulates the frequency, rate, or extent of an immunoglobulin mediated immune response. Relationships: is a type of regulation of B cell mediated immunity [GO:0002712]; regulates immunoglobulin mediated immune response [GO:0016064] Subtypes: regulation of type III hypersensitivity [GO:0001803], GO:0001810, negative regulation of immunoglobulin mediated immune response [GO:0002890], GO:0002891, regulation of type II hypersensitivity [GO:0002892], regulation of humoral immune response mediated by circulating immunoglobulin [GO:0002923], GO:0045191, regulation of immunoglobulin production in mucosal tissue [GO:2000557] Sources: GOC:add